proboscis development [GO:0048728] (BP) Relationships: is a type of animal organ development [GO:0048513]; is part of GO:0035213 Sources: GOC:rc Definition: The process whose specific outcome is the progression of the proboscis over time, from its formation to the mature structure.